mitotic DNA replication lagging strand elongation [GO:1903459] (biological process) Relationships: is a type of lagging strand elongation [GO:0006273]; is a type of DNA strand elongation involved in mitotic DNA replication [GO:1902983] Also known as: lagging strand elongation involved in DNA replication involved in S phase involved in mitotic cell cycle, lagging strand elongation involved in DNA replication involved in S-phase involved in mitotic cell cycle, lagging strand elongation involved in mitotic DNA replication, lagging strand elongation involved in mitotic nuclear cell cycle DNA replication, lagging strand elongation involved in DNA replication during S phase involved in mitotic cell cycle, lagging strand elongation involved in nuclear cell cycle DNA replication involved in mitotic cell cycle Definition: Any lagging strand elongation that is involved in mitotic cell cycle DNA replication. References: PMID:1234 Sources: GOC:TermGenie, GOC:mtg_cell_cycle, GO_REF:0000060